{
  "gene_name": "Tyrosine-protein kinase HCK",
  "term_label": "plasma membrane",
  "gene_symbol": "HCK",
  "term_id": "GO:0005886",
  "gene": "UniProtKB:P08631"
}